{
  "term_label": "collagen catabolic process",
  "term_id": "GO:0030574",
  "gene_symbol": "MMP11",
  "gene_name": "Stromelysin-3",
  "gene": "UniProtKB:P24347"
}